{
  "gene": "UniProtKB:Q9P0T7",
  "gene_name": "Proton-transporting V-type ATPase complex assembly regulator TMEM9",
  "gene_symbol": "TMEM9",
  "term_id": "UNKNOWN:0003",
  "term_label": "Unknown cellular component"
}